{
  "term_label": "Unknown biological process",
  "gene_name": "Olfactory receptor 4F15",
  "gene": "UniProtKB:Q8NGB8",
  "gene_symbol": "OR4F15",
  "term_id": "UNKNOWN:0002"
}